{
  "term_label": "Unknown molecular function",
  "gene_symbol": "CBY3",
  "term_id": "UNKNOWN:0001",
  "gene": "UniProtKB:A6NI87",
  "gene_name": "Protein chibby homolog 3"
}